{
  "gene_symbol": "KRTAP10-5",
  "gene": "UniProtKB:P60370",
  "gene_name": "Keratin-associated protein 10-5",
  "term_label": "Unknown cellular component",
  "term_id": "UNKNOWN:0003"
}